{
  "term_id": "UNKNOWN:0001",
  "term_label": "Unknown molecular function",
  "gene": "UniProtKB:P0C5K7",
  "gene_symbol": "CT62",
  "gene_name": "Cancer_testis antigen 62"
}